{
  "gene_symbol": "ST6GAL1",
  "gene": "UniProtKB:P15907",
  "gene_name": "Beta-galactoside alpha-2,6-sialyltransferase 1",
  "term_label": "Golgi apparatus",
  "term_id": "GO:0005794"
}